{
  "gene_symbol": "NDN",
  "term_label": "Unknown molecular function",
  "gene_name": "Necdin",
  "term_id": "UNKNOWN:0001",
  "gene": "UniProtKB:Q99608"
}